U12-type catalytic step 2 spliceosome [GO:0071018] (cellular component) Definition: A spliceosomal complex that contains the U12, U5 and U6atac snRNPs bound to a splicing intermediate in which the first catalytic cleavage of the 5' splice site has occurred. The precise subunit composition differs significantly from that of the catalytic step 1, or activated, spliceosome, and includes many proteins in addition to those found in the U12, U5 and U6atac snRNPs. References: PMID:16201866 Sources: GOC:ab, GOC:krc, GOC:mah, ISBN:0879695897, ISBN:0879697393 Also known as: minor catalytic step 2 spliceosome, AT-AC catalytic step 2 spliceosome, mammalian U12-type spliceosomal complex C, mammalian U12-type spliceosomal complex C1, yeast U12-type spliceosomal complex A2-2 Relationships: is a type of U12-type spliceosomal complex [GO:0005689]; is a type of catalytic step 2 spliceosome [GO:0071013]; has part U6atac snRNP [GO:0005691]; has part U12 snRNP [GO:0005693]